{
  "term_id": "GO:0120094",
  "gene_symbol": "CDY1B",
  "gene_name": "Testis-specific chromodomain protein Y 1",
  "gene": "UniProtKB:Q9Y6F8",
  "term_label": "negative regulation of peptidyl-lysine crotonylation"
}